fimbrial usher porin activity [GO:0015473] (molecular function) Relationships: is a type of porin activity [GO:0015288] Sources: TC:1.B.11.-.- Definition: A porin that acts in the assembly of fimbria together with fimbrial chaperone.